{
  "term_id": "GO:0007186",
  "gene_name": "Olfactory receptor 5M3",
  "gene": "UniProtKB:Q8NGP4",
  "term_label": "G protein-coupled receptor signaling pathway",
  "gene_symbol": "OR5M3"
}